{
  "term_label": "Unknown cellular component",
  "gene": "UniProtKB:Q5SNV9",
  "term_id": "UNKNOWN:0003",
  "gene_symbol": "C1orf167",
  "gene_name": "Uncharacterized protein C1orf167"
}